{
  "term_id": "GO:0005739",
  "gene_name": "ATP synthase mitochondrial F1 complex assembly factor 2",
  "gene_symbol": "ATPAF2",
  "term_label": "mitochondrion",
  "gene": "UniProtKB:Q8N5M1"
}